{
  "gene": "UniProtKB:O76014",
  "gene_name": "Keratin, type I cuticular Ha7",
  "gene_symbol": "KRT37",
  "term_label": "cytoskeleton",
  "term_id": "GO:0005856"
}